{
  "gene_name": "Cell adhesion molecule DSCAML1",
  "gene": "UniProtKB:Q8TD84",
  "term_label": "homophilic cell-cell adhesion",
  "gene_symbol": "DSCAML1",
  "term_id": "GO:0007156"
}